{
  "gene_name": "Zinc finger protein 35",
  "gene_symbol": "ZNF35",
  "term_label": "regulation of transcription by RNA polymerase II",
  "term_id": "GO:0006357",
  "gene": "UniProtKB:P13682"
}